{
  "gene_name": "Cadherin-10",
  "term_id": "GO:0034332",
  "gene_symbol": "CDH10",
  "gene": "UniProtKB:Q9Y6N8",
  "term_label": "adherens junction organization"
}